negative regulation of male mating behavior [GO:1902436] (biological process) References: PMID:24089208 Sources: GOC:TermGenie Definition: Any process that stops, prevents or reduces the frequency, rate or extent of male mating behavior. Also known as: down regulation of male mating behavior, down-regulation of male mating behavior, downregulation of male mating behavior, inhibition of male mating behavior Relationships: is a type of negative regulation of behavior [GO:0048521]; is a type of regulation of male mating behavior [GO:1902435]; is a type of negative regulation of reproductive process [GO:2000242]; negatively regulates male mating behavior [GO:0060179] Subtypes: negative regulation of turning behavior involved in mating [GO:0061096]